{
  "term_label": "nucleus",
  "gene": "UniProtKB:Q8N8L2",
  "gene_symbol": "ZNF491",
  "term_id": "GO:0005634",
  "gene_name": "Zinc finger protein 491"
}